{
  "gene_symbol": "DNM1L",
  "gene_name": "Dynamin-1-like protein",
  "term_id": "GO:0005737",
  "gene": "UniProtKB:O00429",
  "term_label": "cytoplasm"
}